{
  "gene": "UniProtKB:Q6GMV2",
  "term_id": "GO:0042799",
  "term_label": "histone H4K20 methyltransferase activity",
  "gene_symbol": "SMYD5",
  "gene_name": "Histone-lysine N-trimethyltransferase SMYD5"
}